fatty acid elongation, saturated fatty acid [GO:0019367] (biological process) Relationships: is a type of GO:0030497 Sources: GOC:mah Definition: Elongation of a saturated fatty acid chain.